{
  "term_id": "GO:0061860",
  "gene_name": "Replication factor C subunit 1",
  "gene": "UniProtKB:P35251",
  "term_label": "DNA clamp unloader activity",
  "gene_symbol": "RFC1"
}